{
  "gene_symbol": "LRP3",
  "term_id": "GO:0005886",
  "gene_name": "Low-density lipoprotein receptor-related protein 3",
  "term_label": "plasma membrane",
  "gene": "UniProtKB:O75074"
}